positive regulation of endothelial tube morphogenesis [GO:1905956] (biological process) Definition: Any process that activates or increases the frequency, rate or extent of endothelial tube morphogenesis. Also known as: up regulation of endothelial tube morphogenesis, up-regulation of endothelial tube morphogenesis, upregulation of endothelial tube morphogenesis, activation of endothelial tube morphogenesis Relationships: is a type of positive regulation of multicellular organismal process [GO:0051240]; is a type of regulation of endothelial tube morphogenesis [GO:1901509]; is a type of positive regulation of morphogenesis of an epithelium [GO:1905332]; positively regulates endothelial tube morphogenesis [GO:0061154] References: PMID:25961718 Sources: GOC:BHF, GOC:BHF_miRNA, GOC:TermGenie, GOC:rph, GO_REF:0000058